{
  "gene_symbol": "FFAR3",
  "gene": "UniProtKB:O14843",
  "gene_name": "Free fatty acid receptor 3",
  "term_id": "GO:0071398",
  "term_label": "cellular response to fatty acid"
}